{
  "gene_symbol": "MICALL1",
  "term_id": "GO:0032456",
  "gene": "UniProtKB:Q8N3F8",
  "term_label": "endocytic recycling",
  "gene_name": "MICAL-like protein 1"
}